{
  "term_id": "GO:0005615",
  "term_label": "extracellular space",
  "gene_name": "Lymphotoxin-beta",
  "gene": "UniProtKB:Q06643",
  "gene_symbol": "LTB"
}